{
  "gene": "UniProtKB:Q9UBC5",
  "term_id": "GO:0007605",
  "gene_name": "Unconventional myosin-Ia",
  "gene_symbol": "MYO1A",
  "term_label": "sensory perception of sound"
}